{
  "gene_symbol": "MRPL10",
  "gene": "UniProtKB:Q7Z7H8",
  "term_label": "translation",
  "gene_name": "Large ribosomal subunit protein uL10m",
  "term_id": "GO:0006412"
}